{
  "gene": "UniProtKB:Q96JK9",
  "term_label": "transcription coactivator activity",
  "gene_name": "Mastermind-like protein 3",
  "gene_symbol": "MAML3",
  "term_id": "GO:0003713"
}